negative regulation of CD40 signaling pathway [GO:2000349] (biological process) Definition: Any process that stops, prevents or reduces the frequency, rate or extent of signaling via the CD40 signaling pathway. Sources: GOC:BHF, GOC:mah Also known as: negative regulation of CD40 signalling pathway Relationships: is a type of negative regulation of signal transduction [GO:0009968]; is a type of GO:2000348; negatively regulates CD40 signaling pathway [GO:0023035]